{
  "gene": "UniProtKB:Q8TF01",
  "gene_symbol": "PNISR",
  "term_id": "UNKNOWN:0002",
  "gene_name": "Arginine_serine-rich protein PNISR",
  "term_label": "Unknown biological process"
}